{
  "gene_name": "Olfactory receptor 1E2",
  "term_label": "plasma membrane",
  "term_id": "GO:0005886",
  "gene_symbol": "OR1E2",
  "gene": "UniProtKB:P47887"
}